{
  "term_label": "regulation of inflammatory response",
  "term_id": "GO:0050727",
  "gene_name": "B-cell CLL_lymphoma 6 member B protein",
  "gene_symbol": "BCL6B",
  "gene": "UniProtKB:Q8N143"
}